{
  "term_label": "stereocilium",
  "term_id": "GO:0032420",
  "gene": "UniProtKB:O75838",
  "gene_symbol": "CIB2",
  "gene_name": "Calcium and integrin-binding family member 2"
}